{
  "term_label": "liver development",
  "term_id": "GO:0001889",
  "gene_symbol": "MET",
  "gene_name": "Hepatocyte growth factor receptor",
  "gene": "UniProtKB:P08581"
}